{
  "term_label": "spindle pole",
  "gene": "UniProtKB:Q8NHV4",
  "gene_name": "Protein NEDD1",
  "gene_symbol": "NEDD1",
  "term_id": "GO:0000922"
}